symbiont-mediated suppression of host defenses [GO:0044414] (biological process) Relationships: is a type of symbiont-mediated perturbation of host defenses [GO:0030682] Definition: A process in which a symbiont interferes with, inhibits or disrupts the normal execution of host defense(s) by active mechanisms that normally result in the shutting down of a host pathway. The host is defined as the larger of the organisms involved in a symbiotic interaction. Subtypes: symbiont-mediated suppression of host resistance gene-dependent defense response [GO:0033660], symbiont-mediated suppression of host ethylene-mediated defense response [GO:0052005], GO:0141059, GO:0141154 Sources: GOC:curators Also known as: suppression of defenses of other organism involved in symbiotic interaction, down regulation by symbiont of host defense response, down-regulation by symbiont of host defense response, downregulation by symbiont of host defense response, negative regulation by organism of defense response of other organism involved in symbiotic interaction, negative regulation by symbiont of host defense response, negative regulation of host defenses, suppression of defense response of other organism, suppression of host defense response, suppression of host defenses by symbiont, inhibition by organism of defense response of other organism during symbiotic interaction, inhibition by symbiont of host defense response, down regulation by organism of defense response of other organism during symbiotic interaction, down-regulation by organism of defense response of other organism during symbiotic interaction, downregulation by organism of defense response of other organism during symbiotic interaction, negative regulation by organism of defense response of other organism during symbiotic interaction, suppression of defense response of other organism involved in symbiotic interaction